otic vesicle development [GO:0071599] (biological process) Relationships: is a type of GO:0007423; is a type of tube development [GO:0035295]; is a type of GO:0048839; is a type of GO:0060429 Definition: The process whose specific outcome is the progression of the otic vesicle over time, from its formation to the mature structure. The otic vesicle is a transient embryonic structure formed during development of the vertebrate inner ear. Sources: GOC:mah